enterobactin catabolic process [GO:0046214] (biological process) Also known as: enterobactin breakdown, enterobactin catabolism, enterobactin degradation Relationships: is a type of catechol-containing compound catabolic process [GO:0019614]; is a type of GO:0030640; is a type of macrolide metabolic process [GO:0033067]; is a type of GO:0046215; is a type of lactone catabolic process [GO:1901335] Definition: The chemical reactions and pathways resulting in the breakdown of enterobactin, a catechol-derived siderochrome of Enterobacteria; enterobactin (N',N',N''-(2,6,10-trioxo-1,5,9-triacyclodecane-3,7,11-triyl)tris(2,3-dihydroxy)benzamide) is a self-triester of 2,3-dihydroxy-N-benzoyl-L-serine and a product of the shikimate pathway. Sources: GOC:ai